{
  "gene_name": "Microtubule nucleation factor SSNA1",
  "term_label": "Unknown molecular function",
  "gene_symbol": "SSNA1",
  "gene": "UniProtKB:O43805",
  "term_id": "UNKNOWN:0001"
}